glutamate dehydrogenase (NADP+) activity [GO:0004354] (molecular function) Relationships: is a type of glutamate dehydrogenase [NAD(P)+] activity [GO:0004353] Also known as: L-glutamate dehydrogenase, glutamic acid dehydrogenase, glutamic dehydrogenase activity, L-glutamate:NADP+ oxidoreductase (deaminating), L-glutamic acid dehydrogenase activity, NAD(P)-glutamate dehydrogenase activity, NAD(P)H-dependent glutamate dehydrogenase activity, dehydrogenase, glutamate (nicotinamide adenine dinucleotide (phosphate)) Sources: EC:1.4.1.4 Note: Note that this term has a MetaCyc pathway reference as the pathway only has a single step. Definition: Catalysis of the reaction: L-glutamate + H2O + NADP+ = 2-oxoglutarate + NH3 + NADPH + H+.